{
  "gene_symbol": "TRIM37",
  "term_id": "GO:0006513",
  "term_label": "protein monoubiquitination",
  "gene": "UniProtKB:O94972",
  "gene_name": "E3 ubiquitin-protein ligase TRIM37"
}